{
  "term_label": "plasma membrane",
  "gene_symbol": "CEACAM19",
  "gene": "UniProtKB:Q7Z692",
  "term_id": "GO:0005886",
  "gene_name": "Carcinoembryonic antigen-related cell adhesion molecule 19"
}